{
  "gene_name": "Hemoglobin subunit beta",
  "term_label": "oxygen carrier activity",
  "term_id": "GO:0005344",
  "gene": "UniProtKB:P68871",
  "gene_symbol": "HBB"
}